{
  "gene_name": "Zinc finger protein 425",
  "gene_symbol": "ZNF425",
  "gene": "UniProtKB:Q6IV72",
  "term_id": "GO:0006357",
  "term_label": "regulation of transcription by RNA polymerase II"
}